ribonuclease activator activity [GO:0170054] (molecular function) Definition: Binds to and increases the activity of a ribonuclease. Relationships: is a type of nuclease activator activity [GO:0170053]; positively regulates RNA nuclease activity [GO:0004540] References: PMID:24736845 Also known as: RNA nuclease activator activity Subtypes: exoribonuclease activator activity [GO:0044692], RNA lariat debranching enzyme activator activity [GO:0061632]